{
  "gene_symbol": "PPP1R1B",
  "term_label": "cytoplasm",
  "term_id": "GO:0005737",
  "gene": "UniProtKB:Q9UD71",
  "gene_name": "Protein phosphatase 1 regulatory subunit 1B"
}